{
  "gene_name": "Glucagon-like peptide 2 receptor",
  "gene": "UniProtKB:O95838",
  "term_id": "GO:0017046",
  "term_label": "peptide hormone binding",
  "gene_symbol": "GLP2R"
}